{
  "term_label": "sulfotransferase activity",
  "term_id": "GO:0008146",
  "gene_symbol": "UST",
  "gene": "UniProtKB:Q9Y2C2",
  "gene_name": "Uronyl 2-sulfotransferase"
}